{
  "term_id": "GO:0017171",
  "gene_name": "Valacyclovir hydrolase",
  "gene": "UniProtKB:Q86WA6",
  "term_label": "serine hydrolase activity",
  "gene_symbol": "BPHL"
}